{
  "gene": "UniProtKB:O94822",
  "term_label": "ubiquitin protein ligase activity",
  "gene_name": "E3 ubiquitin-protein ligase listerin",
  "gene_symbol": "LTN1",
  "term_id": "GO:0061630"
}